{
  "gene_symbol": "OCR1",
  "term_id": "UNKNOWN:0003",
  "gene_name": "Ovarian cancer-related protein 1",
  "term_label": "Unknown cellular component",
  "gene": "UniProtKB:Q9BZK8"
}